{
  "gene_symbol": "ZNF8",
  "gene": "UniProtKB:P17098",
  "gene_name": "Zinc finger protein 8",
  "term_label": "nucleus",
  "term_id": "GO:0005634"
}